cation binding [GO:0043169] (molecular function) Sources: GOC:jl Relationships: is a type of ion binding [GO:0043167] Subtypes: GO:0016208, glycine binding [GO:0016594], spermidine binding [GO:0019809], putrescine binding [GO:0019810], cocaine binding [GO:0019811], thiamine binding [GO:0030975], thiamine pyrophosphate binding [GO:0030976], GO:0031210, choline binding [GO:0033265], GO:0034618, dopamine binding [GO:0035240], acetylcholine binding [GO:0042166], GO:0046872, serotonin binding [GO:0051378], GO:0051379, norepinephrine binding [GO:0051380], histamine binding [GO:0051381], GO:0070280, pyridoxamine binding [GO:0070281], ammonium ion binding [GO:0070405], L-leucine binding [GO:0070728], GO:0070905, GO:0072545, tryptophan binding [GO:0120284], proton binding [GO:1901691], L-cysteine binding [GO:1902485], S-adenosyl-L-methionine binding [GO:1904047], chitosan binding [GO:2001080] Definition: Binding to a cation, a charged atom or group of atoms with a net positive charge.